regulation of skeletal muscle tissue growth [GO:0048631] (biological process) Relationships: is a type of GO:0048638; RO_0002211 skeletal muscle tissue growth [GO:0048630] Definition: Any process that modulates the frequency, rate or extent of skeletal muscle growth. References: PMID:15726494, PMID:15907921 Sources: GOC:lm Subtypes: negative regulation of skeletal muscle tissue growth [GO:0048632], positive regulation of skeletal muscle tissue growth [GO:0048633]